{
  "term_label": "RNA transmembrane transporter activity",
  "gene_name": "SID1 transmembrane family member 2",
  "gene_symbol": "SIDT2",
  "gene": "UniProtKB:Q8NBJ9",
  "term_id": "GO:0051033"
}